{
  "gene": "UniProtKB:Q8N3A8",
  "gene_name": "Protein mono-ADP-ribosyltransferase PARP8",
  "gene_symbol": "PARP8",
  "term_label": "kinase binding",
  "term_id": "GO:0019900"
}